ethanolamine ammonia-lyase complex [GO:0009350] (cellular component) Relationships: is_a GO:0140535; is a type of catalytic complex [GO:1902494] References: PMID:1550360 Definition: An enzyme complex that catalyzes the breakdown of ethanolamine to form acetaldehyde and ammonia.